specification of plant organ axis polarity [GO:0090708] (biological process) Definition: The process in which the polarity of a plant organ axis is specified. Sources: GOC:tb Relationships: is a type of specification of axis polarity [GO:0065001]; is part of GO:1905392